{
  "gene": "UniProtKB:Q9UPV9",
  "term_id": "GO:0047496",
  "gene_name": "Trafficking kinesin-binding protein 1",
  "term_label": "vesicle transport along microtubule",
  "gene_symbol": "TRAK1"
}